{
  "term_label": "negative regulation of ERK1 and ERK2 cascade",
  "term_id": "GO:0070373",
  "gene_name": "Sprouty-related, EVH1 domain-containing protein 3",
  "gene_symbol": "SPRED3",
  "gene": "UniProtKB:Q2MJR0"
}